{
  "term_label": "retinoic acid catabolic process",
  "gene": "UniProtKB:Q6V0L0",
  "gene_name": "Cytochrome P450 26C1",
  "term_id": "GO:0034653",
  "gene_symbol": "CYP26C1"
}